post-embryonic camera-type eye morphogenesis [GO:0048597] (biological process) Sources: GOC:jid, GOC:mtg_transport, ISBN:0815340729 Relationships: is a type of post-embryonic eye morphogenesis [GO:0048050]; is part of post-embryonic camera-type eye development [GO:0031077]; is part of GO:0048593 Also known as: post-embryonic eye morphogenesis, post-embryonic camera-style eye morphogenesis Definition: The process in which the anatomical structures of the eye are generated and organized during post-embryonic development.